mesoderm morphogenesis [GO:0048332] (BP) Subtypes: axial mesoderm morphogenesis [GO:0048319], GO:0048340, GO:0048369, intermediate mesoderm morphogenesis [GO:0048390] Relationships: is a type of tissue morphogenesis [GO:0048729]; is part of mesoderm development [GO:0007498] Definition: The process in which the anatomical structures of the mesoderm are generated and organized. Sources: GOC:go_curators